{
  "term_label": "regulation of Notch signaling pathway",
  "term_id": "GO:0008593",
  "gene_symbol": "NEURL1",
  "gene_name": "E3 ubiquitin-protein ligase NEURL1",
  "gene": "UniProtKB:O76050"
}